oxygen carrier activity [GO:0005344] (molecular function) Definition: Binding to oxygen and delivering it to an acceptor molecule or a specific location. Relationships: is a type of molecular carrier activity [GO:0140104]; is part of oxygen transport [GO:0015671]; BFO_0000051 oxygen binding [GO:0019825] Sources: GOC:ai Also known as: globin, hemerythrin, hemocyanin, oxygen-carrying